{
  "gene_name": "Elongation of very long chain fatty acids protein 5",
  "gene_symbol": "ELOVL5",
  "gene": "UniProtKB:Q9NYP7",
  "term_id": "GO:0042761",
  "term_label": "very long-chain fatty acid biosynthetic process"
}